calcium-independent cell-cell adhesion [GO:0016338] (BP) Regulation: regulated by GO:0051040; positively regulated by GO:0051041; negatively regulated by negative regulation of calcium-independent cell-cell adhesion [GO:0051042] Sources: GOC:hb Relationships: is a type of cell-cell adhesion [GO:0098609] Also known as: calcium-independent cell adhesion molecule activity Definition: The attachment of one cell to another cell via adhesion molecules that do not require the presence of calcium for the interaction.